response to cold [GO:0009409] (BP) Also known as: freezing tolerance Subtypes: cold acclimation [GO:0009631], vernalization response [GO:0010048], GO:0050826, cellular response to cold [GO:0070417] Definition: Any process that results in a change in state or activity of a cell or an organism (in terms of movement, secretion, enzyme production, gene expression, etc.) as a result of a cold stimulus, a temperature stimulus below the optimal temperature for that organism. Relationships: is a type of response to stress [GO:0006950]; is a type of response to temperature stimulus [GO:0009266] Sources: GOC:lr